phosphatidylcholine lysophospholipase activity [GO:0004622] (molecular function) Relationships: is_a GO:0120558 Also known as: lysophospholipase activity, 2-lysophosphatidylcholine acylhydrolase activity, lecithinase B activity, lecitholipase activity, lysolecithinase activity, lysophopholipase L2, lysophosphatidase activity, lysophosphatidylcholine hydrolase activity, lysophospholipase A1, phosphatidase B, phospholipase B activity Definition: Catalysis of the reaction: a 1-acyl-sn-glycero-3-phosphocholine + H2O = a fatty acid + H+ + sn-glycerol 3-phosphocholine. Sources: RHEA:15177